ADA complex [GO:0140671] (cellular component) Definition: A chromatin remodeling complex that regulates transcription via acetylation primarily of nucleosomal histones H3 and H2B. In budding yeast shares the histone acetylation (HAT) module of ADA2-GCN5-NGG1-SGF29 with the related SAGA complex. Relationships: is a type of SAGA-type complex [GO:0070461] References: PMID:21734642, PMID:28966424 Sources: GOC:bhm Also known as: ADA HAT complex, ADA histone acetyltransferase complex, scADA, Ada2/Gcn5/Ada3 transcription activator complex